{
  "gene_symbol": "BCO2",
  "term_label": "carotene catabolic process",
  "gene": "UniProtKB:Q9BYV7",
  "gene_name": "Carotenoid-cleaving dioxygenase, mitochondrial",
  "term_id": "GO:0016121"
}